negative regulation of mitotic spindle elongation (spindle phase three) [GO:0110163] (biological process) Definition: Any process that stops, prevents or reduces the frequency, rate or extent of the cell cycle process in which the distance is lengthened between poles of the mitotic spindle during mitotic anaphase B (spindle phase three). Relationships: is_a negative regulation of cytoskeleton organization [GO:0051494]; is a type of regulation of mitotic spindle elongation (spindle phase three) [GO:0110162]; is a type of negative regulation of mitotic spindle elongation [GO:1902845]; negatively regulates mitotic spindle elongation (spindle phase three) [GO:0061805] References: PMID:27697865 Sources: GOC:vw